positive regulation of erythrocyte apoptotic process [GO:1902252] (biological process) Also known as: positive regulation of RBC apoptotic process, positive regulation of red blood cell apoptotic process, up regulation of RBC apoptotic process, up regulation of erythrocyte apoptotic process, up regulation of red blood cell apoptotic process, up-regulation of RBC apoptotic process, up-regulation of erythrocyte apoptotic process, up-regulation of red blood cell apoptotic process, upregulation of RBC apoptotic process, upregulation of erythrocyte apoptotic process, upregulation of red blood cell apoptotic process, activation of RBC apoptosis, activation of RBC apoptotic process, activation of erythrocyte apoptosis, activation of erythrocyte apoptotic process, activation of red blood cell apoptosis, activation of red blood cell apoptotic process, positive regulation of RBC apoptosis, positive regulation of erythrocyte apoptosis, positive regulation of red blood cell apoptosis, up regulation of RBC apoptosis, up regulation of erythrocyte apoptosis, up regulation of red blood cell apoptosis, up-regulation of RBC apoptosis, up-regulation of erythrocyte apoptosis, up-regulation of red blood cell apoptosis, upregulation of RBC apoptosis, upregulation of erythrocyte apoptosis, upregulation of red blood cell apoptosis References: PMID:14569084 Sources: GOC:BHF, GOC:TermGenie, GOC:mtg_apoptosis, GOC:rl Relationships: is a type of positive regulation of myeloid cell apoptotic process [GO:0033034]; is_a regulation of erythrocyte apoptotic process [GO:1902250]; positively regulates erythrocyte apoptotic process [GO:1902217] Definition: Any process that activates or increases the frequency, rate or extent of erythrocyte apoptotic process.